{
  "term_label": "membrane raft",
  "gene_symbol": "CD24",
  "gene": "UniProtKB:P25063",
  "term_id": "GO:0045121",
  "gene_name": "Signal transducer CD24"
}